cellular response to fibroblast growth factor stimulus [GO:0044344] (biological process) Relationships: is a type of cellular response to growth factor stimulus [GO:0071363]; is a type of GO:0071774 Definition: Any process that results in a change in state or activity of a cell (in terms of movement, secretion, enzyme production, gene expression, etc.) as a result of an fibroblast growth factor stimulus. Sources: GOC:jl, GOC:yaf Also known as: cellular response to FGF stimulus